{
  "gene_name": "GS homeobox 2",
  "gene_symbol": "GSX2",
  "gene": "UniProtKB:Q9BZM3",
  "term_label": "nucleus",
  "term_id": "GO:0005634"
}